{
  "gene_symbol": "ATP6V1B1",
  "gene_name": "V-type proton ATPase subunit B, kidney isoform",
  "gene": "UniProtKB:P15313",
  "term_id": "GO:0000221",
  "term_label": "vacuolar proton-transporting V-type ATPase, V1 domain"
}